{
  "gene_symbol": "PPM1D",
  "term_label": "Unknown cellular component",
  "gene_name": "Protein phosphatase 1D",
  "gene": "UniProtKB:O15297",
  "term_id": "UNKNOWN:0003"
}